{
  "gene_symbol": "PRR4",
  "term_id": "UNKNOWN:0003",
  "gene_name": "Proline-rich protein 4",
  "gene": "UniProtKB:Q16378",
  "term_label": "Unknown cellular component"
}